{
  "term_id": "UNKNOWN:0001",
  "gene": "UniProtKB:O95182",
  "gene_name": "NADH dehydrogenase [ubiquinone] 1 alpha subcomplex subunit 7",
  "term_label": "Unknown molecular function",
  "gene_symbol": "NDUFA7"
}